{
  "term_label": "thiamine pyrophosphate transmembrane transporter activity",
  "term_id": "GO:0090422",
  "gene_symbol": "SLC44A4",
  "gene": "UniProtKB:Q53GD3",
  "gene_name": "Choline transporter-like protein 4"
}